negative regulation of cholesterol efflux [GO:0090370] (biological process) Definition: Any process that decreases the frequency, rate or extent of cholesterol efflux. Cholesterol efflux is the directed movement of cholesterol, cholest-5-en-3-beta-ol, out of a cell or organelle. Sources: GOC:dph, GOC:tb, GOC:yaf Relationships: is a type of regulation of cholesterol efflux [GO:0010874]; is_a negative regulation of cholesterol transport [GO:0032375]; negatively regulates cholesterol efflux [GO:0033344]